{
  "term_label": "Unknown biological process",
  "gene_name": "V-type proton ATPase subunit E 2",
  "gene": "UniProtKB:Q96A05",
  "gene_symbol": "ATP6V1E2",
  "term_id": "UNKNOWN:0002"
}